endexine [GO:0043671] (cellular component) Relationships: is a type of GO:0110165; BFO_0000050 GO:0043668 Definition: The inner part of the exine, which stains. Note: Note that endexine is distinguished on staining properties; compare with 'sexine ; GO:0043673'. See also 'ectexine ; GO:0043669'. References: PMID:28904424